epithelial cilium movement involved in extracellular fluid movement [GO:0003351] (biological process) Definition: The directed, self-propelled movement of cilia of epithelial cells. Depending on the type of cell, there may be one or many cilia per cell. This movement is usually coordinated between many epithelial cells, and serves to move extracellular fluid. Sources: GOC:dph, GOC:krc Also known as: cilium movement involved in fluid flow, epithelial cilium beating Relationships: is a type of cilium movement [GO:0003341]; is a type of extracellular transport [GO:0006858]; is a type of GO:0099111 Subtypes: cilium movement involved in otolith formation [GO:0003355], epithelial cilium movement involved in determination of left/right asymmetry [GO:0060287], cerebrospinal fluid circulation [GO:0090660], mucociliary clearance [GO:0120197]